{
  "gene": "UniProtKB:Q9C019",
  "term_id": "GO:0005737",
  "term_label": "cytoplasm",
  "gene_symbol": "TRIM15",
  "gene_name": "E3 ubiquitin-protein ligase TRIM15"
}